{
  "gene_name": "Vesicular glutamate transporter 1",
  "gene_symbol": "SLC17A7",
  "term_id": "GO:0050803",
  "term_label": "regulation of synapse structure or activity",
  "gene": "UniProtKB:Q9P2U7"
}